{
  "term_id": "GO:0045499",
  "gene_symbol": "SEMA3F",
  "gene": "UniProtKB:Q13275",
  "gene_name": "Semaphorin-3F",
  "term_label": "chemorepellent activity"
}